{
  "gene_symbol": "TNFSF13B",
  "gene": "UniProtKB:Q9Y275",
  "gene_name": "Tumor necrosis factor ligand superfamily member 13B",
  "term_id": "GO:0030890",
  "term_label": "positive regulation of B cell proliferation"
}